{
  "term_id": "GO:0016239",
  "term_label": "positive regulation of macroautophagy",
  "gene": "UniProtKB:Q6ZNE9",
  "gene_symbol": "RUFY4",
  "gene_name": "RUN and FYVE domain-containing protein 4"
}